{
  "gene_name": "Coiled-coil domain-containing protein 125",
  "term_label": "negative regulation of Rho protein signal transduction",
  "term_id": "GO:0035024",
  "gene": "UniProtKB:Q86Z20",
  "gene_symbol": "CCDC125"
}